stabilization of membrane potential [GO:0030322] (biological process) Definition: The accomplishment of a non-fluctuating membrane potential, the electric potential existing across any membrane arising from charges in the membrane itself and from the charges present in the media on either side of the membrane. Relationships: is a type of regulation of membrane potential [GO:0042391] Sources: GOC:jl, ISBN:0198506732